{
  "term_id": "GO:0004725",
  "gene": "UniProtKB:P08575",
  "gene_name": "Receptor-type tyrosine-protein phosphatase C",
  "gene_symbol": "PTPRC",
  "term_label": "protein tyrosine phosphatase activity"
}